{
  "term_label": "phospholipid dephosphorylation",
  "term_id": "GO:0046839",
  "gene": "UniProtKB:Q9BX95",
  "gene_name": "Sphingosine-1-phosphate phosphatase 1",
  "gene_symbol": "SGPP1"
}